{
  "gene_symbol": "NUCKS1",
  "term_label": "cytoplasm",
  "gene": "UniProtKB:Q9H1E3",
  "gene_name": "Nuclear ubiquitous casein and cyclin-dependent kinase substrate 1",
  "term_id": "GO:0005737"
}